cycloheximide:proton antiporter activity [GO:0015309] (molecular function) Relationships: is a type of proton transmembrane transporter activity [GO:0015078]; is a type of cycloheximide transmembrane transporter activity [GO:0015243]; is a type of antiporter activity [GO:0015297] Sources: TC:2.A.1.2.2 Also known as: cycloheximide:hydrogen antiporter activity Definition: Enables the transfer of a solute or solutes from one side of a membrane to the other according to the reaction: H+(out) + cycloheximide(in) = H+(in) + cycloheximide(out).